fat-soluble vitamin catabolic process [GO:0042363] (biological process) Also known as: fat-soluble vitamin breakdown, fat-soluble vitamin catabolism, fat-soluble vitamin degradation Definition: The chemical reactions and pathways resulting in the breakdown of any of a diverse group of vitamins that are soluble in organic solvents and relatively insoluble in water. Relationships: is a type of vitamin catabolic process [GO:0009111] Subtypes: GO:0034653, GO:0042369, vitamin K catabolic process [GO:0042377] Sources: GOC:jl, ISBN:0198506732